D5 dopamine receptor binding [GO:0031752] (molecular function) Also known as: D1B dopamine receptor binding, D5 dopamine receptor ligand Relationships: is a type of GO:0050780 Definition: Binding to a D5 dopamine receptor. Sources: GOC:mah, GOC:nln